{
  "gene_symbol": "MAGT1",
  "term_id": "GO:0018279",
  "gene": "UniProtKB:Q9H0U3",
  "term_label": "protein N-linked glycosylation via asparagine",
  "gene_name": "Magnesium transporter protein 1"
}